piRNA dual-strand cluster binding [GO:1990472] (MF) Relationships: is a type of piRNA cluster binding [GO:1990470] References: PMID:24906153 Sources: GOC:bhm Definition: Binding to dual-strand piRNA clusters, double-stranded DNA regions that give rise to PIWI-interacting RNAs (piRNAs) where piRNAs originate from both DNA strands via noncanonical transcription. Note: An example of this is rhi in Drosophila melanogaster (Q7JXA8) in PMID:24906153 (inferred from direct assay).